{
  "gene_name": "Mediator of RNA polymerase II transcription subunit 22",
  "gene": "UniProtKB:Q15528",
  "term_label": "Unknown molecular function",
  "gene_symbol": "MED22",
  "term_id": "UNKNOWN:0001"
}